cytosol pyruvate dehydrogenase (lipoamide) phosphatase complex [GO:0045249] (cellular component) References: PMID:9395502 Sources: GOC:mtg_sensu Relationships: is a type of pyruvate dehydrogenase (lipoamide) phosphatase complex [GO:0045253]; is part of cytosol [GO:0005829] Note: See also the cellular component term 'cytosolic pyruvate dehydrogenase complex ; GO:0045250'. Definition: A cytosolic complex of a regulatory and catalytic subunit that catalyzes the dephosphorylation and concomitant reactivation of the alpha subunit of the E1 component of the pyruvate dehydrogenase complex.